{
  "gene": "UniProtKB:P10415",
  "gene_symbol": "BCL2",
  "term_label": "mitochondrial outer membrane",
  "gene_name": "Apoptosis regulator Bcl-2",
  "term_id": "GO:0005741"
}